positive regulation of acetylcholine uptake [GO:0051633] (biological process) Definition: Any process that activates or increases the frequency, rate or extent of the directed movement of acetylcholine into a cell. Sources: GOC:ai Also known as: positive regulation of acetylcholine import, up regulation of acetylcholine uptake, up-regulation of acetylcholine uptake, upregulation of acetylcholine uptake, activation of acetylcholine uptake, stimulation of acetylcholine uptake Relationships: is a type of regulation of acetylcholine uptake [GO:0051631]; is a type of positive regulation of amine transport [GO:0051954]; positively regulates acetylcholine uptake [GO:0051630]